branching involved in submandibular gland morphogenesis [GO:1990632] (biological process) Also known as: submandibular gland branching morphogenesis, submandibular gland ductal branching Relationships: is a type of branching involved in salivary gland morphogenesis [GO:0060445] Definition: The process in which the branching structure of the submandibular gland is generated and organized. References: PMID:15063181, PMID:20890964